blood vessel endothelial cell delamination involved in blood vessel lumen ensheathment [GO:1902354] (biological process) Definition: Any blood vessel endothelial cell delamination that is involved in blood vessel lumen ensheathment. References: PMID:23698350 Sources: GOC:TermGenie, GOC:dgh Relationships: is a type of GO:0097497; is part of GO:0097496